{
  "gene_symbol": "FOSL1",
  "term_label": "DNA-binding transcription factor activity, RNA polymerase II-specific",
  "term_id": "GO:0000981",
  "gene_name": "Fos-related antigen 1",
  "gene": "UniProtKB:P15407"
}